regulation of fucose catabolic process [GO:0043468] (biological process) Sources: GOC:mlg Relationships: is a type of regulation of carbohydrate catabolic process [GO:0043470]; is_a regulation of small molecule metabolic process [GO:0062012]; regulates fucose catabolic process [GO:0019317] Definition: Any process that modulates the frequency, rate, or extent of the chemical reactions and pathways resulting in the breakdown of fucose.